regulation of calcineurin-mediated signaling [GO:0106056] (biological process) References: PMID:25081204 Relationships: is a type of regulation of calcium-mediated signaling [GO:0050848]; regulates calcineurin-mediated signaling [GO:0097720] Definition: Any process that modulates the frequency, rate or extent of calcineurin-mediated signaling. Subtypes: regulation of calcineurin-NFAT signaling cascade [GO:0070884], GO:0106057, GO:0106058